{
  "gene_name": "Pleckstrin homology domain-containing family G member 5",
  "gene_symbol": "PLEKHG5",
  "gene": "UniProtKB:O94827",
  "term_id": "GO:0005886",
  "term_label": "plasma membrane"
}